regulation of vascular associated smooth muscle cell differentiation [GO:1905063] (biological process) Also known as: regulation of VSMC differentiation, regulation of vascular smooth muscle cell differentiation References: PMID:19088079 Sources: GOC:BHF, GOC:BHF_miRNA, GOC:TermGenie, GOC:rph, GO_REF:0000058 Definition: Any process that modulates the frequency, rate or extent of vascular smooth muscle cell differentiation. Subtypes: GO:1904829, GO:1905064, GO:1905065, regulation of vascular associated smooth muscle cell differentiation involved in phenotypic switching [GO:1905930], regulation of cardiac vascular smooth muscle cell differentiation [GO:2000722] Relationships: is a type of regulation of smooth muscle cell differentiation [GO:0051150]; regulates GO:0035886